positive regulation of chemokine (C-X-C motif) ligand 2 production [GO:2000343] (biological process) Sources: GOC:BHF, GOC:mah Definition: Any process that activates or increases the frequency, rate or extent of chemokine (C-X-C motif) ligand 2 production. Also known as: positive regulation of CCL2 secretion, positive regulation of CXCL2 production, positive regulation of MIP-2 production, positive regulation of MIP2 production, positive regulation of SCYB2 production, positive regulation of chemokine (C-C motif) ligand 2 secretion Relationships: is a type of positive regulation of chemokine production [GO:0032722]; is a type of regulation of chemokine (C-X-C motif) ligand 2 production [GO:2000341]; positively regulates chemokine (C-X-C motif) ligand 2 production [GO:0072567]